{
  "gene_name": "Zinc finger protein 771",
  "term_label": "nucleus",
  "gene": "UniProtKB:Q7L3S4",
  "term_id": "GO:0005634",
  "gene_symbol": "ZNF771"
}